pantoate 4-dehydrogenase activity [GO:0050166] (molecular function) Relationships: is a type of oxidoreductase activity, acting on the CH-OH group of donors, NAD or NADP as acceptor [GO:0016616] Definition: Catalysis of the reaction: (R)-pantoate + NAD+ = (R)-4-dehydropantoate + H+ + NADH. Sources: EC:1.1.1.106, RHEA:23000 Also known as: (R)-pantoate:NAD+ 4-oxidoreductase activity, D-pantoate:NAD+ 4-oxidoreductase activity, panthothenase activity, pantoate dehydrogenase activity